{
  "term_label": "diadenosine hexaphosphate catabolic process",
  "term_id": "GO:1901909",
  "gene_symbol": "NUDT11",
  "gene_name": "Diphosphoinositol polyphosphate phosphohydrolase 3-beta",
  "gene": "UniProtKB:Q96G61"
}